{
  "term_label": "metalloendopeptidase activity",
  "gene_name": "Meprin A subunit beta",
  "gene": "UniProtKB:Q16820",
  "term_id": "GO:0004222",
  "gene_symbol": "MEP1B"
}